{
  "gene": "UniProtKB:Q8NB59",
  "gene_name": "Synaptotagmin-14",
  "gene_symbol": "SYT14",
  "term_id": "GO:0005543",
  "term_label": "phospholipid binding"
}